{
  "gene": "UniProtKB:P22304",
  "term_id": "GO:0005764",
  "gene_symbol": "IDS",
  "term_label": "lysosome",
  "gene_name": "Iduronate 2-sulfatase"
}